sperm end piece [GO:0097229] (CC) Definition: The short tip of the sperm flagellum, adjacent to the sperm principal piece and furthest from the sperm head, which contains only the axoneme surrounded by the plasma membrane. Sources: GOC:cjm, GOC:sart, MP:0009837 Relationships: is a type of GO:0110165; is part of sperm flagellum [GO:0036126]